riboflavinase activity [GO:0050258] (molecular function) Definition: Catalysis of the reaction: H2O + H+ + riboflavin = D-ribitol + lumichrome. Also known as: riboflavin hydrolase activity Sources: EC:3.5.99.1, RHEA:11408 Relationships: is a type of hydrolase activity, acting on carbon-nitrogen (but not peptide) bonds [GO:0016810]